{
  "gene_name": "T cell receptor alpha joining 16 (Fragment)",
  "gene": "UniProtKB:A0A075B6V0",
  "term_label": "Unknown biological process",
  "term_id": "UNKNOWN:0002",
  "gene_symbol": "TRAJ16"
}